negative regulation of imaginal disc growth [GO:0045571] (biological process) Also known as: down regulation of imaginal disc growth, down-regulation of imaginal disc growth, downregulation of imaginal disc growth, inhibition of imaginal disc growth Relationships: is a type of GO:0045570; is a type of negative regulation of developmental growth [GO:0048640]; negatively regulates imaginal disc growth [GO:0007446] Definition: Any process that stops, prevents, or reduces the frequency, rate or extent of imaginal disc growth. Sources: GOC:go_curators